{
  "term_id": "UNKNOWN:0002",
  "gene": "UniProtKB:Q96JB8",
  "gene_name": "MAGUK p55 subfamily member 4",
  "term_label": "Unknown biological process",
  "gene_symbol": "MPP4"
}